chemoattraction of branchiomotor neuron axon in branchial arch mesenchyme [GO:0021791] (biological process) Definition: The process in which a branchiomotor neuron growth cone in the branchial arch mesenchyme is directed to a specific target site in the branchial arch mesenchyme in response to an attractive chemical cue. Branchiomotor neurons are located in the hindbrain and innervate branchial arch-derived muscles that control jaw movements, facial expression, the larynx, and the pharynx. References: PMID:14699587 Sources: GOC:cls, GOC:dgh, GOC:dph, GOC:jid, GO_REF:0000021 Also known as: positive chemotaxis of branchiomotor neuron axon in branchial arch mesenchyme Relationships: is a type of GO:0021789; is a type of GO:0021792